{
  "gene": "UniProtKB:Q5T890",
  "gene_symbol": "ERCC6L2",
  "term_label": "Unknown cellular component",
  "term_id": "UNKNOWN:0003",
  "gene_name": "DNA excision repair protein ERCC-6-like 2"
}